{
  "term_label": "neuron differentiation",
  "gene_symbol": "RTN1",
  "gene_name": "Reticulon-1",
  "term_id": "GO:0030182",
  "gene": "UniProtKB:Q16799"
}